{
  "gene": "UniProtKB:Q92887",
  "gene_symbol": "ABCC2",
  "term_id": "GO:0016324",
  "gene_name": "ATP-binding cassette sub-family C member 2",
  "term_label": "apical plasma membrane"
}